tolerance induction to lipopolysaccharide [GO:0072573] (biological process) Also known as: tolerance induction to endotoxin, tolerance induction to LPS Sources: GOC:BHF, GOC:mah Relationships: is a type of tolerance induction [GO:0002507]; is_a GO:0031665; BFO_0000050 GO:0071222 Definition: Tolerance induction directed at lipopolysaccharide antigens.